{
  "gene": "UniProtKB:Q15615",
  "gene_name": "Olfactory receptor 4D1",
  "gene_symbol": "OR4D1",
  "term_label": "Unknown biological process",
  "term_id": "UNKNOWN:0002"
}